{
  "term_label": "positive regulation of canonical Wnt signaling pathway",
  "term_id": "GO:0090263",
  "gene_symbol": "PPM1N",
  "gene_name": "Probable protein phosphatase 1N",
  "gene": "UniProtKB:Q8N819"
}